{
  "gene_name": "Carnitine O-palmitoyltransferase 1, brain isoform",
  "gene_symbol": "CPT1C",
  "term_label": "carnitine metabolic process",
  "gene": "UniProtKB:Q8TCG5",
  "term_id": "GO:0009437"
}